{
  "term_label": "negative regulation of gene expression, epigenetic",
  "term_id": "GO:0045814",
  "gene_name": "Metal-response element-binding transcription factor 2",
  "gene_symbol": "MTF2",
  "gene": "UniProtKB:Q9Y483"
}